{
  "term_id": "GO:0005938",
  "gene_name": "Tubulin-folding cofactor B",
  "gene_symbol": "TBCB",
  "gene": "UniProtKB:Q99426",
  "term_label": "cell cortex"
}